{
  "term_id": "GO:0005737",
  "term_label": "cytoplasm",
  "gene_symbol": "TMCO1",
  "gene_name": "Calcium load-activated calcium channel",
  "gene": "UniProtKB:Q9UM00"
}